{
  "term_id": "GO:0016525",
  "gene": "UniProtKB:P07996",
  "gene_name": "Thrombospondin-1",
  "term_label": "negative regulation of angiogenesis",
  "gene_symbol": "THBS1"
}